{
  "gene_symbol": "TMPRSS11A",
  "gene_name": "Transmembrane protease serine 11A",
  "term_label": "protein processing",
  "gene": "UniProtKB:Q6ZMR5",
  "term_id": "GO:0016485"
}